lavandulyl diphosphate synthase activity [GO:0033851] (molecular function) Definition: Catalysis of the reaction: 2 dimethylallyl diphosphate = diphosphate + lavandulyl diphosphate. Sources: EC:2.5.1.69, RHEA:21676 Also known as: FDS-5, dimethylallyl-diphosphate:dimethylallyl-diphosphate dimethylallyltransferase (lavandulyl-diphosphate-forming) activity Relationships: is a type of transferase activity, transferring alkyl or aryl (other than methyl) groups [GO:0016765]